{
  "term_label": "regulation of apoptotic process",
  "gene": "UniProtKB:P39687",
  "term_id": "GO:0042981",
  "gene_name": "Acidic leucine-rich nuclear phosphoprotein 32 family member A",
  "gene_symbol": "ANP32A"
}